{
  "gene_symbol": "NTAN1",
  "gene": "UniProtKB:Q96AB6",
  "term_id": "GO:0005634",
  "term_label": "nucleus",
  "gene_name": "Protein N-terminal asparagine amidohydrolase"
}